C/EBP complex [GO:1990647] (cellular component) Definition: A dimeric, sequence specific DNA-binding transcription factor complex regulating the expression of genes involved in immune and inflammatory responses. Exists at least as alpha and beta homodimeric forms. Binds to regulatory regions of several acute-phase and cytokines genes and probably plays a role in the regulation of acute-phase reaction, inflammation and hemopoiesis. The consensus recognition site is 5'-T[TG]NNGNAA[TG]-3'. Transcription factor activity is inhibited by binding of CHOP forming heterodimers with alternative transcription factor activities. References: PMID:8657121 Sources: GOC:PARL, GOC:bhm, GOC:pad Note: An example of this is Cebpa in rat (P05554) in PMID:8657121 (inferred from direct assay). Also known as: C/EBP homodimer complex, C/EBP transcription factor complex, C/EBPalpha complex, C/EBPalpha homodimer complex, C/EBPbeta complex, C/EBPbeta homodimer complex Relationships: is a type of RNA polymerase II transcription regulator complex [GO:0090575]